{
  "gene_symbol": "Q6ZS49",
  "gene_name": "Putative uncharacterized protein FLJ45831",
  "gene": "UniProtKB:Q6ZS49",
  "term_label": "Unknown molecular function",
  "term_id": "UNKNOWN:0001"
}